nucleotide-sugar transmembrane transporter activity [GO:0005338] (molecular function) Subtypes: pyrimidine nucleotide-sugar transmembrane transporter activity [GO:0015165], purine nucleotide-sugar transmembrane transporter activity [GO:0036080] References: PMID:15034926 Sources: GOC:ai, GOC:mtg_transport, ISBN:0815340729 Relationships: is a type of organophosphate ester transmembrane transporter activity [GO:0015605]; is a type of nucleobase-containing compound transmembrane transporter activity [GO:0015932]; is a type of carbohydrate derivative transmembrane transporter activity [GO:1901505] Definition: Enables the transfer of a nucleotide-sugar from one side of a membrane to the other. A nucleotide-sugar is any nucleotide in which the distal phosphoric residue of a nucleoside 5'-diphosphate is in glycosidic linkage with a monosaccharide or monosaccharide derivative.